negative regulation of cellulose catabolic process [GO:2000998] (biological process) Sources: GOC:mengo_curators Also known as: negative regulation of cellulose breakdown, negative regulation of cellulose catabolism, negative regulation of cellulose degradation Relationships: is a type of negative regulation of catabolic process [GO:0009895]; is a type of negative regulation of macromolecule metabolic process [GO:0010605]; is a type of negative regulation of carbohydrate metabolic process [GO:0045912]; is a type of regulation of cellulose catabolic process [GO:2000997]; negatively regulates cellulose catabolic process [GO:0030245] Definition: Any process that stops, prevents or reduces the frequency, rate or extent of cellulose catabolic process.